positive regulation of tumor necrosis factor-mediated signaling pathway [GO:1903265] (biological process) Relationships: is a type of positive regulation of cytokine-mediated signaling pathway [GO:0001961]; is a type of regulation of tumor necrosis factor-mediated signaling pathway [GO:0010803]; positively regulates tumor necrosis factor-mediated signaling pathway [GO:0033209] Also known as: positive regulation of tumor necrosis factor-mediated signalling pathway, up regulation of tumor necrosis factor-mediated signaling pathway, up regulation of tumor necrosis factor-mediated signalling pathway, up-regulation of tumor necrosis factor-mediated signaling pathway, up-regulation of tumor necrosis factor-mediated signalling pathway, upregulation of tumor necrosis factor-mediated signaling pathway, upregulation of tumor necrosis factor-mediated signalling pathway, activation of TNF-alpha-mediated signaling pathway, activation of tumor necrosis factor alpha-mediated signaling pathway, activation of tumor necrosis factor-mediated signaling pathway, activation of tumor necrosis factor-mediated signalling pathway, positive regulation of TNF-alpha-mediated signaling pathway, positive regulation of tumor necrosis factor alpha-mediated signaling pathway, up regulation of TNF-alpha-mediated signaling pathway, up regulation of tumor necrosis factor alpha-mediated signaling pathway, up-regulation of TNF-alpha-mediated signaling pathway, up-regulation of tumor necrosis factor alpha-mediated signaling pathway, upregulation of TNF-alpha-mediated signaling pathway, upregulation of tumor necrosis factor alpha-mediated signaling pathway, activation of adipocytokine signaling pathway, positive regulation of adipocytokine signaling pathway, up regulation of adipocytokine signaling pathway, up-regulation of adipocytokine signaling pathway, upregulation of adipocytokine signaling pathway Definition: Any process that activates or increases the frequency, rate or extent of tumor necrosis factor-mediated signaling pathway. References: PMID:23453807 Sources: GOC:PARL, GOC:TermGenie, GOC:bf, GO_REF:0000058